XY body [GO:0001741] (cellular component) Definition: A structure found in a male mammalian spermatocyte containing an unpaired X chromosome that has become densely heterochromatic, silenced and localized at the nuclear periphery. References: PMID:20622855 Sources: GOC:hjd, GOC:mr, Wikipedia:XY_sex-determination_system Relationships: is a type of sex chromosome [GO:0000803]; has part condensed chromatin of inactivated sex chromosome [GO:0098578]